galactoglucomannan catabolic process [GO:2000885] (biological process) Relationships: is a type of polysaccharide catabolic process [GO:0000272]; is_a galactoglucomannan metabolic process [GO:0010392] Also known as: galactoglucomannan catabolism Definition: The chemical reactions and pathways resulting in the breakdown of a galactoglucomannan. Sources: GOC:mengo_curators Regulation: regulated by GO:2000912; negatively regulated by negative regulation of galactoglucomannan catabolic process [GO:2000913]; positively regulated by positive regulation of galactoglucomannan catabolic process [GO:2000914]